{
  "term_label": "axonogenesis",
  "gene": "UniProtKB:P46821",
  "term_id": "GO:0007409",
  "gene_symbol": "MAP1B",
  "gene_name": "Microtubule-associated protein 1B"
}